left ventricular cardiac muscle tissue morphogenesis [GO:0003220] (biological process) Relationships: is_a ventricular cardiac muscle tissue morphogenesis [GO:0055010]; is part of cardiac left ventricle morphogenesis [GO:0003214] Subtypes: GO:0003224, left ventricular trabecular myocardium morphogenesis [GO:0003225] Sources: GOC:mtg_heart Definition: The process in which the anatomical structures of left cardiac ventricle muscle are generated and organized. Also known as: left ventricular myocardium morphogenesis